detection of increased carbon dioxide by carotid body chemoreceptor signaling [GO:0003035] (biological process) Definition: The process in which information about the levels of carbon dioxide are received and are converted to a molecular signal by chemoreceptors in a carotid body. Sources: GOC:mtg_cardio Relationships: is a type of detection of increased carbon dioxide by chemoreceptor signaling [GO:0003021]; is part of detection of hypoxic conditions in blood by carotid body chemoreceptor signaling [GO:0003029] Also known as: detection of increased carbon dioxide by carotid body chemoreceptor signalling